{
  "gene_symbol": "PRSS41",
  "gene": "UniProtKB:Q7RTY9",
  "term_label": "serine-type peptidase activity",
  "term_id": "GO:0008236",
  "gene_name": "Serine protease 41"
}